{
  "term_id": "UNKNOWN:0001",
  "term_label": "Unknown molecular function",
  "gene": "UniProtKB:Q96BT1",
  "gene_name": "Putative uncharacterized protein C3orf49",
  "gene_symbol": "C3orf49"
}